{
  "term_id": "GO:0005543",
  "gene_name": "Phospholipase A2 group V",
  "gene_symbol": "PLA2G5",
  "term_label": "phospholipid binding",
  "gene": "UniProtKB:P39877"
}